{
  "term_label": "Unknown molecular function",
  "gene_symbol": "CRB3",
  "term_id": "UNKNOWN:0001",
  "gene": "UniProtKB:Q9BUF7",
  "gene_name": "Protein crumbs homolog 3"
}